{
  "gene_symbol": "ANKRD20A1",
  "term_label": "Unknown cellular component",
  "term_id": "UNKNOWN:0003",
  "gene": "UniProtKB:Q5TYW2",
  "gene_name": "Ankyrin repeat domain-containing protein 20A1"
}